RNA polymerase inhibitor activity [GO:0140870] (molecular function) Relationships: is_a enzyme inhibitor activity [GO:0004857]; RO_0002212 GO:0097747 Regulation: RO_0002212 by repressor of RNA polymerase inhibitor activity [GO:0140871] Definition: Binds to and stops, prevents or reduces the activity of RNA polymerase. References: PMID:15300239, PMID:18313387, PMID:31048766